{
  "term_id": "UNKNOWN:0002",
  "gene_name": "Uncharacterized protein DKFZp434B061",
  "gene_symbol": "Q9UF83",
  "term_label": "Unknown biological process",
  "gene": "UniProtKB:Q9UF83"
}